{
  "gene_name": "Kinesin-like protein KIF3A",
  "term_label": "cytoplasm",
  "gene": "UniProtKB:Q9Y496",
  "gene_symbol": "KIF3A",
  "term_id": "GO:0005737"
}